{
  "term_id": "GO:0051402",
  "gene": "UniProtKB:Q96A26",
  "term_label": "neuron apoptotic process",
  "gene_symbol": "FAM162A",
  "gene_name": "Protein FAM162A"
}